{
  "gene_symbol": "CLDN23",
  "gene": "UniProtKB:Q96B33",
  "term_label": "bicellular tight junction",
  "term_id": "GO:0005923",
  "gene_name": "Claudin-23"
}